{
  "gene_symbol": "LIG3",
  "term_id": "GO:0006302",
  "gene": "UniProtKB:P49916",
  "term_label": "double-strand break repair",
  "gene_name": "DNA ligase 3"
}